arginase activity [GO:0004053] (molecular function) Relationships: is a type of hydrolase activity, acting on carbon-nitrogen (but not peptide) bonds, in linear amidines [GO:0016813] Also known as: L-arginase activity, L-arginine amidinohydrolase activity, arginine amidinase activity, arginine transamidinase activity, canavanase activity Definition: Catalysis of the reaction: L-arginine + H2O = L-ornithine + urea. Sources: EC:3.5.3.1